{
  "term_id": "UNKNOWN:0001",
  "gene_name": "NXPE family member 4",
  "gene": "UniProtKB:Q6UWF7",
  "gene_symbol": "NXPE4",
  "term_label": "Unknown molecular function"
}